{
  "gene": "UniProtKB:Q6PB30",
  "term_id": "UNKNOWN:0003",
  "gene_symbol": "CSAG1",
  "gene_name": "Chondrosarcoma-associated gene 1 protein",
  "term_label": "Unknown cellular component"
}